{
  "term_id": "UNKNOWN:0002",
  "gene": "UniProtKB:Q6UXP7",
  "gene_name": "Protein FAM151B",
  "gene_symbol": "FAM151B",
  "term_label": "Unknown biological process"
}